{
  "gene_name": "E3 ubiquitin-protein ligase RNF31",
  "term_id": "UNKNOWN:0003",
  "gene": "UniProtKB:Q96EP0",
  "gene_symbol": "RNF31",
  "term_label": "Unknown cellular component"
}